{
  "gene_name": "Protein tyrosine phosphatase domain-containing protein 1",
  "term_id": "GO:0060271",
  "gene": "UniProtKB:A2A3K4",
  "gene_symbol": "PTPDC1",
  "term_label": "cilium assembly"
}